{
  "term_id": "GO:0005794",
  "term_label": "Golgi apparatus",
  "gene": "UniProtKB:Q8WUA7",
  "gene_name": "TBC1 domain family member 22A",
  "gene_symbol": "TBC1D22A"
}